{
  "gene_name": "Spermatogenesis-associated protein 4",
  "term_id": "GO:0005930",
  "gene": "UniProtKB:Q8NEY3",
  "gene_symbol": "SPATA4",
  "term_label": "axoneme"
}